{
  "gene_symbol": "ZFP92",
  "gene": "UniProtKB:A6NM28",
  "term_label": "RNA polymerase II cis-regulatory region sequence-specific DNA binding",
  "term_id": "GO:0000978",
  "gene_name": "Zinc finger protein 92 homolog"
}